negative regulation of axon regeneration [GO:0048681] (biological process) Sources: GOC:dgh, GOC:dph, GOC:jid, GOC:lm Subtypes: negative regulation of collateral sprouting of intact axon in response to injury [GO:0048685], negative regulation of sprouting of injured axon [GO:0048688], negative regulation of optical nerve axon regeneration [GO:1905592] Definition: Any process that stops, prevents, or reduces the frequency, rate or extent of axon regeneration. Relationships: is a type of GO:0032102; is a type of regulation of axon regeneration [GO:0048679]; is a type of negative regulation of neuron projection regeneration [GO:0070571]; is a type of negative regulation of response to wounding [GO:1903035]; negatively regulates GO:0031103 Also known as: down regulation of axon regeneration, down-regulation of axon regeneration, downregulation of axon regeneration, inhibition of axon regeneration